{
  "gene": "UniProtKB:P01344",
  "gene_name": "Insulin-like growth factor II",
  "term_label": "positive regulation of MAPK cascade",
  "term_id": "GO:0043410",
  "gene_symbol": "IGF2"
}